{
  "term_label": "Golgi apparatus",
  "gene_name": "HEAT repeat-containing protein 5A",
  "gene_symbol": "HEATR5A",
  "term_id": "GO:0005794",
  "gene": "UniProtKB:Q86XA9"
}